proline racemase activity [GO:0018112] (molecular function) Relationships: is a type of GO:0047661 Definition: Catalysis of the reaction: L-proline = D-proline. Sources: EC:5.1.1.4, RHEA:10680